protein-heme P460 linkage [GO:0018174] (biological process) Also known as: protein-haem P460 linkage Sources: RESID:AA0266, RESID:AA0271 Relationships: is a type of protein-heme linkage [GO:0017003]; is a type of cytochrome complex assembly [GO:0017004] Definition: The linkage of protein to heme P460.